{
  "term_label": "RNA polymerase II cis-regulatory region sequence-specific DNA binding",
  "gene_name": "Peroxisome proliferator-activated receptor alpha",
  "gene": "UniProtKB:Q07869",
  "gene_symbol": "PPARA",
  "term_id": "GO:0000978"
}